{
  "gene_symbol": "MROH8",
  "term_label": "Unknown cellular component",
  "gene": "UniProtKB:Q9H579",
  "term_id": "UNKNOWN:0003",
  "gene_name": "Protein MROH8"
}